{
  "term_label": "cytoplasm",
  "gene": "UniProtKB:Q9NZW4",
  "gene_name": "Dentin sialophosphoprotein",
  "term_id": "GO:0005737",
  "gene_symbol": "DSPP"
}